{
  "gene_name": "Polycomb group RING finger protein 1",
  "gene_symbol": "PCGF1",
  "gene": "UniProtKB:Q9BSM1",
  "term_label": "negative regulation of transcription by RNA polymerase II",
  "term_id": "GO:0000122"
}